{
  "term_label": "regulation of transcription by RNA polymerase II",
  "gene_name": "Zinc finger and BTB domain-containing protein 43",
  "term_id": "GO:0006357",
  "gene": "UniProtKB:O43298",
  "gene_symbol": "ZBTB43"
}